negative regulation of protein processing [GO:0010955] (biological process) Definition: Any process that decreases the rate, frequency or extent of protein maturation by peptide bond cleavage. Sources: GOC:dph, GOC:mah, GOC:tb Also known as: negative regulation of protein maturation by peptide bond cleavage Relationships: is_a negative regulation of proteolysis [GO:0045861]; is a type of GO:0070613; is a type of GO:1903318; RO_0002212 protein processing [GO:0016485] Subtypes: negative regulation of plasminogen activation [GO:0010757], negative regulation of peptide hormone processing [GO:0060570], zymogen inhibition [GO:0097341], negative regulation of protein processing involved in protein targeting to mitochondrion [GO:1903217], negative regulation of protein processing in phagocytic vesicle [GO:1903922]